{
  "gene": "UniProtKB:P01574",
  "gene_name": "Interferon beta",
  "gene_symbol": "IFNB1",
  "term_label": "T cell activation involved in immune response",
  "term_id": "GO:0002286"
}